distal axon [GO:0150034] (cellular component) Definition: That part of an axon close to and including the growth cone or the axon terminus. Relationships: is_a GO:0110165; is part of axon [GO:0030424] Also known as: distal part of axon, distal part of the axon References: PMID:17202468 Sources: GOC:aruk, GOC:bc